response to meiotic recombination checkpoint signaling [GO:0072461] (biological process) Definition: A process that occurs in response to signals generated as a result of meiotic recombination checkpoint signaling. Sources: GOC:mtg_cell_cycle Also known as: meiotic recombination checkpoint effector process, response to signal involved in meiotic recombination checkpoint Relationships: is a type of response to meiotic cell cycle checkpoint signaling [GO:0072410]; is a type of meiotic cell cycle process [GO:1903046]; is part of meiotic recombination checkpoint signaling [GO:0051598]